{
  "term_id": "UNKNOWN:0003",
  "gene_name": "Lysine-rich coiled-coil protein 1",
  "gene": "UniProtKB:Q9NPI7",
  "term_label": "Unknown cellular component",
  "gene_symbol": "KRCC1"
}